{
  "term_label": "immunoglobulin complex",
  "term_id": "GO:0019814",
  "gene_name": "Immunoglobulin lambda variable 2-14",
  "gene_symbol": "IGLV2-14",
  "gene": "UniProtKB:P01704"
}